succinate metabolic process [GO:0006105] (biological process) Definition: The chemical reactions and pathways involving succinate, also known as butanedioate or ethane dicarboxylate, the dianion of succinic acid. Succinate is an important intermediate in metabolism and a component of the TCA cycle. Also known as: succinate metabolism Sources: ISBN:0198506732 Relationships: is a type of dicarboxylic acid metabolic process [GO:0043648] Subtypes: GO:0006540, L-arginine catabolic process to succinate [GO:0019545], GO:0019657, mixed acid fermentation [GO:0019664]